xyloglucan-specific exo-beta-1,4-glucanase activity [GO:0033950] (molecular function) Also known as: Cel74A, [(1->6)-alpha-D-xylo]-(1->4)-beta-D-glucan exo-glucohydrolase activity Definition: Catalysis of the reaction: xyloglucan + H2O = xyloglucan oligosaccharides. This reaction is the exohydrolysis of 1,4-beta-D-glucosidic linkages in xyloglucan. Sources: EC:3.2.1.155 Relationships: is_a beta-glucanase activity [GO:0052736]